negative regulation of chemokine (C-C motif) ligand 4 production [GO:0071644] (biological process) Relationships: is a type of negative regulation of chemokine production [GO:0032682]; is a type of regulation of chemokine (C-C motif) ligand 4 production [GO:0071643]; negatively regulates chemokine (C-C motif) ligand 4 production [GO:0071606] Definition: Any process that stops, prevents, or reduces the frequency, rate, or extent of production of chemokine (C-C motif) ligand 4. Also known as: negative regulation of macrophage inflammatory protein production, negative regulation of CCL4 production, negative regulation of MIP-1b production Sources: GOC:mah